{
  "gene_name": "Selenoprotein W",
  "term_id": "GO:0030218",
  "gene": "UniProtKB:P63302",
  "gene_symbol": "SELENOW",
  "term_label": "erythrocyte differentiation"
}